{
  "gene": "UniProtKB:A6NIE6",
  "gene_name": "Putative RRN3-like protein RRN3P2",
  "gene_symbol": "RRN3P2",
  "term_id": "GO:0001042",
  "term_label": "RNA polymerase I core binding"
}